linear element assembly [GO:0030999] (biological process) References: PMID:30640914 Sources: GOC:jb, GOC:mah Also known as: linear element formation Definition: The cell cycle process in which linear elements are assembled in association with fission yeast chromosomes during meiotic prophase. Linear element assembly begins with LinE complex formation and ends when LinE complexes are associated with chromatin in structures visible as nuclear foci. A linear element is a proteinaceous scaffold related to the synaptonemal complex. Regulation: regulated by regulation of linear element assembly [GO:0090006] Relationships: is a type of cellular component assembly [GO:0022607]; is_a meiotic cell cycle process [GO:1903046]; is part of homologous chromosome pairing at meiosis [GO:0007129]